{
  "term_label": "proteoglycan biosynthetic process",
  "term_id": "GO:0030166",
  "gene_symbol": "CHST13",
  "gene_name": "Carbohydrate sulfotransferase 13",
  "gene": "UniProtKB:Q8NET6"
}